{
  "gene_symbol": "CAMK1",
  "term_label": "signal transduction",
  "gene": "UniProtKB:Q14012",
  "gene_name": "Calcium_calmodulin-dependent protein kinase type 1",
  "term_id": "GO:0007165"
}